{
  "gene_name": "Vesicle-associated membrane protein 4",
  "gene_symbol": "VAMP4",
  "term_label": "presynaptic endosome membrane",
  "term_id": "GO:0098954",
  "gene": "UniProtKB:O75379"
}